'de novo' GMP biosynthetic process [GO:0106387] (biological process) Also known as: 'de novo' guanosine 5'-monophosphate biosynthetic process References: PMID:25605736 Definition: The chemical reactions and pathways resulting in the formation of guanosine 5'-monophosphate (GMP) through an inosine 5'-monophosphate (IMP) intermediate. Relationships: is a type of GMP biosynthetic process [GO:0006177]